glucosyltransferase activity [GO:0046527] (molecular function) Sources: ISBN:0198506732 Definition: Catalysis of the transfer of a glucosyl group to an acceptor molecule, typically another carbohydrate or a lipid. Subtypes: dolichyl-phosphate-glucose-glycolipid alpha-glucosyltransferase activity [GO:0004583], GO:0016759, xyloglucan:xyloglucosyl transferase activity [GO:0016762], 1,4-alpha-glucan 6-alpha-glucosyltransferase activity [GO:0032001], DNA alpha-glucosyltransferase activity [GO:0033820], DNA beta-glucosyltransferase activity [GO:0033821], glucosyl-DNA beta-glucosyltransferase activity [GO:0033822], procollagen glucosyltransferase activity [GO:0033823], oligosaccharide 4-alpha-D-glucosyltransferase activity [GO:0033825], GO:0033826, GO:0033828, GO:0033831, GO:0033832, flavonol 7-O-beta-glucosyltransferase activity [GO:0033836], GO:0033837, flavonol-3-O-glucoside glucosyltransferase activity [GO:0033838], flavonol-3-O-glycoside glucosyltransferase activity [GO:0033839], alpha-1,4-glucan glucosyltransferase (NDP-glucose donor) activity [GO:0033840], GO:0035251, protein-arginine rhamnosyltransferase activity [GO:0106361] Relationships: is a type of hexosyltransferase activity [GO:0016758]